{
  "gene": "UniProtKB:Q14117",
  "term_label": "cytosol",
  "term_id": "GO:0005829",
  "gene_symbol": "DPYS",
  "gene_name": "Dihydropyrimidinase"
}